{
  "gene": "UniProtKB:Q96SQ5",
  "term_label": "RNA polymerase II cis-regulatory region sequence-specific DNA binding",
  "gene_symbol": "ZNF587",
  "term_id": "GO:0000978",
  "gene_name": "Zinc finger protein 587"
}